{
  "term_label": "plasma membrane",
  "term_id": "GO:0005886",
  "gene_name": "Olfactory receptor 13H1",
  "gene": "UniProtKB:Q8NG92",
  "gene_symbol": "OR13H1"
}